glucose-1-phosphate cytidylyltransferase activity [GO:0047343] (molecular function) Definition: Catalysis of the reaction: alpha-D-glucose 1-phosphate + CTP = CDP-D-glucose + diphosphate. Sources: RHEA:18213 Also known as: CTP:glucose-1-phosphate cytidylyltransferase activity, CDP glucose pyrophosphorylase activity, CDP-glucose diphosphorylase activity, CDP-glucose pyrophosphorylase activity, CTP:D-glucose-1-phosphate cytidylyltransferase activity, CTP:alpha-D-glucose-1-phosphate cytidylyltransferase activity, cytidine diphosphate glucose pyrophosphorylase activity, cytidine diphosphate-D-glucose pyrophosphorylase activity, cytidine diphosphoglucose pyrophosphorylase activity Relationships: is a type of cytidylyltransferase activity [GO:0070567]